{
  "term_label": "myosin phosphatase regulator activity",
  "gene": "UniProtKB:O14974",
  "term_id": "GO:0017020",
  "gene_name": "Protein phosphatase 1 regulatory subunit 12A",
  "gene_symbol": "PPP1R12A"
}